{
  "gene_name": "Acetylcholine receptor subunit gamma",
  "term_label": "plasma membrane",
  "gene_symbol": "CHRNG",
  "term_id": "GO:0005886",
  "gene": "UniProtKB:P07510"
}